{
  "gene": "UniProtKB:Q9HCL0",
  "gene_symbol": "PCDH18",
  "term_id": "GO:0005886",
  "gene_name": "Protocadherin-18",
  "term_label": "plasma membrane"
}